{
  "term_id": "GO:0000981",
  "gene": "UniProtKB:Q00653",
  "gene_name": "Nuclear factor NF-kappa-B p100 subunit",
  "gene_symbol": "NFKB2",
  "term_label": "DNA-binding transcription factor activity, RNA polymerase II-specific"
}